{
  "term_id": "GO:0015030",
  "gene": "UniProtKB:O75312",
  "gene_name": "Zinc finger protein ZPR1",
  "term_label": "Cajal body",
  "gene_symbol": "ZPR1"
}